endolysosome lumen [GO:0036021] (cellular component) Definition: The volume enclosed by the membrane of an endolysosome. An endolysosome is a transient hybrid organelle formed by fusion of a late endosome with a lysosome. Sources: GOC:pde Also known as: endolysosomal lumen Relationships: is a type of endosome lumen [GO:0031904]; is a type of GO:0043202; is part of GO:0036019